{
  "term_id": "GO:0005254",
  "gene_name": "Gamma-aminobutyric acid receptor subunit alpha-1",
  "gene_symbol": "GABRA1",
  "gene": "UniProtKB:P14867",
  "term_label": "chloride channel activity"
}